negative regulation of gamma-aminobutyric acid secretion [GO:0014053] (biological process) Relationships: is a type of regulation of gamma-aminobutyric acid secretion [GO:0014052]; is a type of negative regulation of organic acid transport [GO:0032891]; is a type of negative regulation of secretion [GO:0051048]; is a type of negative regulation of amino acid transport [GO:0051956]; negatively regulates gamma-aminobutyric acid secretion [GO:0014051] Sources: GOC:ef Also known as: down regulation of gamma-aminobutyric acid secretion, down-regulation of gamma-aminobutyric acid secretion, downregulation of gamma-aminobutyric acid secretion, negative regulation of GABA secretion, inhibition of gamma-aminobutyric acid secretion Definition: Any process that stops, prevents, or reduces the frequency, rate or extent of the regulated release of gamma-aminobutyric acid.